(-)-pinoresinol biosynthetic process [GO:1901599] (biological process) Sources: GOC:TermGenie Also known as: (-)-pinoresinol anabolism, (-)-pinoresinol biosynthesis, (-)-pinoresinol formation, (-)-pinoresinol synthesis Relationships: is a type of lignan biosynthetic process [GO:0009807]; is a type of GO:0046189; is a type of ether biosynthetic process [GO:1901503]; is a type of (-)-pinoresinol metabolic process [GO:1901598] Definition: The chemical reactions and pathways resulting in the formation of (-)-pinoresinol.